{
  "term_id": "GO:0000122",
  "gene": "UniProtKB:Q7Z2F6",
  "gene_name": "KRAB domain-containing protein 5",
  "gene_symbol": "KRBOX5",
  "term_label": "negative regulation of transcription by RNA polymerase II"
}